positive regulation of thrombin-activated receptor signaling pathway [GO:0070496] (biological process) Relationships: is a type of positive regulation of G protein-coupled receptor signaling pathway [GO:0045745]; is a type of GO:0070494; positively regulates thrombin-activated receptor signaling pathway [GO:0070493] Definition: Any process that activates or increases the frequency, rate or extent of thrombin-activated receptor protein signaling pathway activity. A thrombin receptor signaling pathway is the series of molecular signals generated as a consequence of a thrombin-activated receptor binding to one of its physiological ligands. Also known as: positive regulation of thrombin receptor signaling pathway, positive regulation of thrombin receptor signalling pathway Sources: GOC:mah